{
  "gene_name": "C-Jun-amino-terminal kinase-interacting protein 4",
  "term_id": "GO:0008432",
  "term_label": "JUN kinase binding",
  "gene_symbol": "SPAG9",
  "gene": "UniProtKB:O60271"
}